{
  "gene_name": "Synaptotagmin-13",
  "gene_symbol": "SYT13",
  "term_id": "GO:0030424",
  "gene": "UniProtKB:Q7L8C5",
  "term_label": "axon"
}